{
  "gene_name": "Ubiquitin-associated and SH3 domain-containing protein B",
  "term_id": "GO:0045779",
  "term_label": "negative regulation of bone resorption",
  "gene_symbol": "UBASH3B",
  "gene": "UniProtKB:Q8TF42"
}